amino-acid betaine biosynthetic process [GO:0006578] (biological process) Definition: The chemical reactions and pathways resulting in the formation of any betaine, the N-trimethyl derivative of an amino acid. Sources: GOC:mah, ISBN:0198506732 Relationships: is a type of amino-acid betaine metabolic process [GO:0006577]; is a type of modified amino acid biosynthetic process [GO:0042398] Also known as: betaine anabolism, betaine biosynthesis, betaine biosynthetic process, betaine formation, betaine synthesis Subtypes: L-proline betaine biosynthetic process [GO:0019503], glycine betaine biosynthetic process [GO:0031456], carnitine biosynthetic process [GO:0045329], GO:0052699, GO:1903257